{
  "term_label": "cis-regulatory region sequence-specific DNA binding",
  "gene": "UniProtKB:P32314",
  "gene_symbol": "FOXN2",
  "term_id": "GO:0000987",
  "gene_name": "Forkhead box protein N2"
}